{
  "term_label": "nuclear localization sequence binding",
  "gene_name": "Importin subunit alpha-3",
  "gene_symbol": "KPNA4",
  "gene": "UniProtKB:O00629",
  "term_id": "GO:0008139"
}